{
  "gene": "UniProtKB:P09622",
  "gene_name": "Dihydrolipoyl dehydrogenase, mitochondrial",
  "gene_symbol": "DLD",
  "term_id": "GO:0050660",
  "term_label": "flavin adenine dinucleotide binding"
}